{
  "gene_name": "Chorionic somatomammotropin hormone-like 1",
  "gene": "UniProtKB:Q14406",
  "gene_symbol": "CSHL1",
  "term_id": "GO:0046427",
  "term_label": "positive regulation of receptor signaling pathway via JAK-STAT"
}